vagina development [GO:0060068] (biological process) Sources: GOC:dph, GOC:ebc Relationships: is a type of female genitalia development [GO:0030540] Definition: The reproductive developmental process whose specific outcome is the progression of the vagina over time, from its formation to the mature structure.